{
  "term_id": "GO:0043123",
  "gene_symbol": "CARD10",
  "gene": "UniProtKB:Q9BWT7",
  "term_label": "positive regulation of canonical NF-kappaB signal transduction",
  "gene_name": "Caspase recruitment domain-containing protein 10"
}